{
  "gene": "UniProtKB:Q86X27",
  "term_id": "GO:0005085",
  "gene_name": "Ras-specific guanine nucleotide-releasing factor RalGPS2",
  "gene_symbol": "RALGPS2",
  "term_label": "guanyl-nucleotide exchange factor activity"
}